{
  "gene_name": "Immunoglobulin heavy variable 3_OR16-17 (non-functional) (Fragment)",
  "gene": "UniProtKB:S4R3C0",
  "term_label": "antigen binding",
  "gene_symbol": "IGHV3OR16-17",
  "term_id": "GO:0003823"
}